{
  "gene_symbol": "DYNC1H1",
  "gene": "UniProtKB:Q14204",
  "gene_name": "Cytoplasmic dynein 1 heavy chain 1",
  "term_id": "GO:0005868",
  "term_label": "cytoplasmic dynein complex"
}